{
  "gene_name": "BLOC-1-related complex subunit 5",
  "term_id": "GO:0030672",
  "gene": "UniProtKB:Q969J3",
  "term_label": "synaptic vesicle membrane",
  "gene_symbol": "BORCS5"
}